{
  "gene_name": "5'-AMP-activated protein kinase subunit gamma-3",
  "gene_symbol": "PRKAG3",
  "term_label": "protein kinase binding",
  "term_id": "GO:0019901",
  "gene": "UniProtKB:Q9UGI9"
}